establishment of protease localization to T cell secretory granule [GO:0033378] (biological process) Definition: The directed movement of a protease to a location within a secretory granule in a T cell. Relationships: is a type of establishment of protein localization to T cell secretory granule [GO:0033376]; is part of protease localization to T cell secretory granule [GO:0033375] Subtypes: establishment of granzyme B localization to T cell secretory granule [GO:0033381] Also known as: establishment of protease localisation in T cell secretory granule, establishment of protease localization in T cell secretory granule, establishment of protease localization in T lymphocyte secretory granule, establishment of protease localization in T-cell secretory granule, establishment of protease localization in T-lymphocyte secretory granule Sources: GOC:mah